{
  "gene": "UniProtKB:Q96AQ8",
  "term_label": "mitochondrion",
  "term_id": "GO:0005739",
  "gene_symbol": "MCUR1",
  "gene_name": "Mitochondrial calcium uniporter regulator 1"
}